{
  "gene": "UniProtKB:A8MYZ5",
  "gene_symbol": "IQCF6",
  "term_label": "Unknown biological process",
  "term_id": "UNKNOWN:0002",
  "gene_name": "IQ domain-containing protein F6"
}